{
  "gene_name": "C-C motif chemokine 3",
  "gene": "UniProtKB:P10147",
  "term_id": "GO:0070098",
  "term_label": "chemokine-mediated signaling pathway",
  "gene_symbol": "CCL3"
}